{
  "gene_name": "Somatostatin receptor type 3",
  "gene": "UniProtKB:P32745",
  "term_label": "plasma membrane",
  "gene_symbol": "SSTR3",
  "term_id": "GO:0005886"
}